type II transforming growth factor beta receptor binding [GO:0005114] (molecular function) Also known as: TGF-beta type II binding, transforming growth factor beta receptor type II binding, type II TGF-beta binding, punt binding, punt ligand, transforming growth factor beta ligand binding to type II receptor Relationships: is a type of transforming growth factor beta receptor binding [GO:0005160] References: PMID:11252892 Sources: GOC:ceb, GOC:mah Definition: Binding to a type II transforming growth factor beta receptor.